iron incorporation into metallo-sulfur cluster [GO:0018283] (BP) Also known as: iron incorporation into metallo-sulphur cluster Relationships: is a type of GO:0016226; is a type of metal incorporation into metallo-sulfur cluster [GO:0018282] Definition: The incorporation of iron into a metallo-sulfur cluster. Sources: GOC:ai